{
  "term_label": "Unknown molecular function",
  "gene": "UniProtKB:A0A1B0GTH9",
  "gene_symbol": "LOC100505841",
  "gene_name": "Zinc finger protein 474",
  "term_id": "UNKNOWN:0001"
}